xanthosine transport [GO:0015863] (BP) Relationships: is a type of GO:0015858 Sources: ISBN:0198506732 Definition: The directed movement of xanthosine, xanthine riboside, into, out of or within a cell, or between cells, by means of some agent such as a transporter or pore.